{
  "term_id": "GO:0042700",
  "gene_name": "Lutropin subunit beta",
  "gene_symbol": "LHB",
  "gene": "UniProtKB:P01229",
  "term_label": "luteinizing hormone signaling pathway"
}